meiosis I cytokinesis [GO:0007110] (biological process) Sources: GOC:mtg_cell_cycle Definition: A cell cycle process that results in the division of the cytoplasm of a cell after meiosis I, resulting in the separation of the original cell into two daughter cells. Also known as: cytokinesis after meiosis I Relationships: is a type of meiotic cytokinesis [GO:0033206]; is a type of meiosis I cell cycle process [GO:0061982]